{
  "gene_name": "Tudor and KH domain-containing protein",
  "gene": "UniProtKB:Q9Y2W6",
  "term_label": "P granule",
  "term_id": "GO:0043186",
  "gene_symbol": "TDRKH"
}